{
  "term_label": "plasma membrane",
  "gene": "UniProtKB:Q86YT5",
  "gene_symbol": "SLC13A5",
  "gene_name": "Na(+)_citrate cotransporter",
  "term_id": "GO:0005886"
}